Hub1 activating enzyme activity [GO:0042293] (MF) Sources: GOC:mah Definition: Catalysis of the activation of the small ubiquitin-related modifier Hub1, through the formation of an ATP-dependent high-energy thiolester bond. Relationships: is a type of GO:0008641